{
  "gene": "UniProtKB:O76100",
  "term_label": "olfactory receptor activity",
  "gene_name": "Olfactory receptor 7A10",
  "term_id": "GO:0004984",
  "gene_symbol": "OR7A10"
}